{
  "gene": "UniProtKB:Q6P5S7",
  "term_label": "Unknown cellular component",
  "gene_symbol": "RNASEK",
  "gene_name": "Ribonuclease kappa",
  "term_id": "UNKNOWN:0003"
}